{
  "term_id": "GO:0050852",
  "gene": "UniProtKB:O00481",
  "gene_name": "Butyrophilin subfamily 3 member A1",
  "term_label": "T cell receptor signaling pathway",
  "gene_symbol": "BTN3A1"
}